{
  "gene_name": "Nascent polypeptide-associated complex subunit alpha, muscle-specific form",
  "term_id": "GO:0006612",
  "gene": "UniProtKB:E9PAV3",
  "gene_symbol": "NACA",
  "term_label": "protein targeting to membrane"
}